{
  "gene": "UniProtKB:Q6ICH7",
  "gene_name": "Aspartate beta-hydroxylase domain-containing protein 2",
  "term_label": "Unknown cellular component",
  "gene_symbol": "ASPHD2",
  "term_id": "UNKNOWN:0003"
}